{
  "term_id": "GO:0070778",
  "gene_symbol": "SLC1A2",
  "gene": "UniProtKB:P43004",
  "term_label": "L-aspartate transmembrane transport",
  "gene_name": "Excitatory amino acid transporter 2"
}